{
  "term_label": "RNA polymerase II transcription regulatory region sequence-specific DNA binding",
  "gene_name": "Zinc finger protein 619",
  "gene_symbol": "ZNF619",
  "term_id": "GO:0000977",
  "gene": "UniProtKB:Q8N2I2"
}